(R)-2-hydroxy-fatty acid dehydrogenase (NAD+) activity [GO:0047049] (molecular function) Relationships: is a type of GO:0016616 Also known as: 2-hydroxy fatty acid oxidase, (R)-2-hydroxy-fatty-acid dehydrogenase activity, (R)-2-hydroxystearate:NAD+ oxidoreductase activity, D-2-hydroxy fatty acid dehydrogenase activity Sources: EC:1.1.1.98, RHEA:15949 Definition: Catalysis of the reaction: (R)-2-hydroxystearate + NAD+ = 2-oxostearate + H+ + NADH.